mitochondrial oxaloacetate transmembrane transport [GO:1990555] (biological process) Definition: The process in which oxaloacetate is transported across a mitochondrial membrane, into or out of the mitochondrion. Relationships: is a type of GO:1902356 References: PMID:10428783